{
  "gene_symbol": "TBC1D14",
  "term_label": "autophagosome",
  "gene_name": "TBC1 domain family member 14",
  "term_id": "GO:0005776",
  "gene": "UniProtKB:Q9P2M4"
}